CENP-A containing chromatin [GO:0061638] (cellular component) Also known as: centromeric core region chromatin, chromatin containing CENP-A, nuclear CENP-A containing chromatin, centromeric core domain chromatin References: PMID:20206496, PMID:22729156, PMID:24710126 Sources: GOC:vw Definition: The specialized chromatin located in the centromeric core region or the entire centromeric region in organisms with point centromeres, which is enriched for CENP-A-containing nucleosomes. This chromatin forms a 3-dimensional structure which provides a platform for kinetochore assembly and microtubule attachment. Relationships: is a type of GO:0000785; is part of chromosome, centromeric core domain [GO:0034506]